negative regulation of colon smooth muscle contraction [GO:1904342] (biological process) Definition: Any process that stops, prevents or reduces the frequency, rate or extent of colon smooth muscle contraction. References: PMID:24170253 Sources: GOC:TermGenie, GO_REF:0000058 Also known as: down regulation of colon smooth muscle contraction, down-regulation of colon smooth muscle contraction, downregulation of colon smooth muscle contraction, inhibition of colon smooth muscle contraction Relationships: is_a negative regulation of gastro-intestinal system smooth muscle contraction [GO:1904305]; is a type of regulation of colon smooth muscle contraction [GO:1904341]; RO_0002212 GO:1990765